response to butan-1-ol [GO:1901422] (biological process) References: PMID:24014527 Sources: GOC:TermGenie, GOC:mengo_curators Also known as: process resulting in tolerance to butan-1-ol Definition: Any process that results in a change in state or activity of a cell or an organism (in terms of movement, secretion, enzyme production, gene expression, etc.) as a result of a butan-1-ol stimulus. Regulation: RO_0002211 by regulation of response to butan-1-ol [GO:1901448]; negatively regulated by GO:1901449; positively regulated by positive regulation of response to butan-1-ol [GO:1901450] Relationships: is a type of response to lipid [GO:0033993]; is a type of response to alcohol [GO:0097305]